lipid A phosphate methyltransferase activity [GO:0043839] (molecular function) Relationships: is a type of GO:0008757 Definition: Catalysis of the transfer of a methyl group from S-adenosylmethionine (SAM) to the 1-phosphate group of lipid A. References: PMID:15994324 Also known as: lipid A methyltransferase, lipid A 1-phosphomethyltransferase activity, lipid A phosphomethyltransferase activity, LmtA